{
  "term_id": "UNKNOWN:0002",
  "gene": "UniProtKB:Q8NFA0",
  "gene_symbol": "USP32",
  "gene_name": "Ubiquitin carboxyl-terminal hydrolase 32",
  "term_label": "Unknown biological process"
}